{
  "gene_symbol": "MX2",
  "gene": "UniProtKB:P20592",
  "gene_name": "Interferon-induced GTP-binding protein Mx2",
  "term_label": "nucleus",
  "term_id": "GO:0005634"
}